{
  "term_label": "Smc5-Smc6 complex",
  "gene": "UniProtKB:Q8WV22",
  "term_id": "GO:0030915",
  "gene_symbol": "NSMCE1",
  "gene_name": "Non-structural maintenance of chromosomes element 1 homolog"
}